{
  "gene": "UniProtKB:Q8N3X1",
  "gene_symbol": "FNBP4",
  "term_label": "Unknown cellular component",
  "gene_name": "Formin-binding protein 4",
  "term_id": "UNKNOWN:0003"
}